snRNA pseudouridylation guide activity [GO:0030565] (MF) Relationships: is a type of GO:0030558; is a type of GO:0030566 References: PMID:11733745 Note: Note that this term describes the activity of a nucleic acid, usually RNA, gene product that interacts with other RNA molecules via base pairing; it should not be used to annotate proteins. Note that this term may be useful for annotating snoRNAs. Definition: Activity that provides specificity to a pseudouridine synthetase by using base complementarity to guide site-specific pseudouridylations to a small nuclear RNA molecule.